{
  "gene": "UniProtKB:Q5SWH9",
  "gene_symbol": "TMEM69",
  "gene_name": "Transmembrane protein 69",
  "term_id": "UNKNOWN:0002",
  "term_label": "Unknown biological process"
}